{
  "term_label": "regulatory ncRNA-mediated post-transcriptional gene silencing",
  "term_id": "GO:0035194",
  "gene": "UniProtKB:Q9HCK5",
  "gene_name": "Protein argonaute-4",
  "gene_symbol": "AGO4"
}